{
  "gene_symbol": "NPTX2",
  "gene_name": "Neuronal pentraxin-2",
  "term_id": "UNKNOWN:0003",
  "gene": "UniProtKB:P47972",
  "term_label": "Unknown cellular component"
}